{
  "term_id": "GO:1900118",
  "gene_name": "Humanin-like 5",
  "term_label": "negative regulation of execution phase of apoptosis",
  "gene_symbol": "MTRNR2L5",
  "gene": "UniProtKB:P0CJ72"
}